lateral reticular nucleus development [GO:0021726] (biological process) Sources: GOC:cls, GOC:curators, GOC:dgh, GOC:dph, GOC:jid Definition: The process whose specific outcome is the progression of the lateral reticular nucleus over time, from its formation to the mature structure. Relationships: is a type of neural nucleus development [GO:0048857]; is part of medullary reticular formation development [GO:0021723]